{
  "term_id": "UNKNOWN:0003",
  "gene_name": "NHS-like protein 2",
  "gene": "UniProtKB:Q5HYW2",
  "term_label": "Unknown cellular component",
  "gene_symbol": "NHSL2"
}